visceral motor neuron differentiation [GO:0021524] (biological process) Relationships: is a type of spinal cord motor neuron differentiation [GO:0021522] References: PMID:11262869 Sources: GOC:cls, GOC:dgh, GOC:dph, GOC:jid, GO_REF:0000021 Definition: The process in which neuroepithelial cells in the neural tube acquire specialized structural and/or functional features of visceral motor neurons. Visceral motor neurons innervate glandular targets and are responsible for transmission of motor impulses from the brain to the periphery. Differentiation includes the processes involved in commitment of a cell to a specific fate.